{
  "gene_name": "Pecanex-like protein 2",
  "term_id": "UNKNOWN:0003",
  "gene_symbol": "PCNX2",
  "term_label": "Unknown cellular component",
  "gene": "UniProtKB:A6NKB5"
}